ether hydrolase activity [GO:0016803] (molecular function) Relationships: is a type of GO:0016801 Definition: Catalysis of the hydrolysis of an ether bond, -O-. Subtypes: epoxide hydrolase activity [GO:0004301], leukotriene-A4 hydrolase activity [GO:0004463], cholesterol-5,6-oxide hydrolase activity [GO:0033963], alkenylglycerophosphocholine hydrolase activity [GO:0047408], trans-epoxysuccinate hydrolase activity [GO:0050345], mannosylglycerate hydrolase activity [GO:0102546], GO:0102547 Sources: EC:3.3.2.-, GOC:ai